{
  "gene_symbol": "TIMP4",
  "term_id": "GO:0034097",
  "gene": "UniProtKB:Q99727",
  "term_label": "response to cytokine",
  "gene_name": "Metalloproteinase inhibitor 4"
}